{
  "gene": "UniProtKB:P05000",
  "term_label": "adaptive immune response",
  "term_id": "GO:0002250",
  "gene_symbol": "IFNW1",
  "gene_name": "Interferon omega-1"
}